{
  "gene_name": "Glycine receptor subunit alpha-1",
  "term_id": "GO:0005254",
  "gene": "UniProtKB:P23415",
  "gene_symbol": "GLRA1",
  "term_label": "chloride channel activity"
}